{
  "gene_symbol": "RUFY2",
  "term_label": "Unknown biological process",
  "gene": "UniProtKB:Q8WXA3",
  "term_id": "UNKNOWN:0002",
  "gene_name": "RUN and FYVE domain-containing protein 2"
}